{
  "gene_symbol": "FSCB",
  "gene": "UniProtKB:Q5H9T9",
  "gene_name": "Fibrous sheath CABYR-binding protein",
  "term_label": "sperm fibrous sheath",
  "term_id": "GO:0035686"
}